{
  "gene": "UniProtKB:P13804",
  "term_id": "GO:0009055",
  "term_label": "electron transfer activity",
  "gene_name": "Electron transfer flavoprotein subunit alpha, mitochondrial",
  "gene_symbol": "ETFA"
}